phaseollidin hydratase activity [GO:0047454] (molecular function) Definition: Catalysis of the reaction: phaseollidin hydrate = H2O + phaseollidin. Sources: EC:4.2.1.97, RHEA:19769 Also known as: phaseollidin-hydrate hydro-lyase (phaseollidin-forming), phaseollidin-hydrate hydro-lyase activity Relationships: is a type of hydro-lyase activity [GO:0016836]